{
  "term_label": "branched-chain amino acid transport",
  "gene": "UniProtKB:Q96H78",
  "gene_name": "Solute carrier family 25 member 44",
  "gene_symbol": "SLC25A44",
  "term_id": "GO:0015803"
}